{
  "term_label": "norepinephrine:sodium symporter activity",
  "gene": "UniProtKB:P23975",
  "term_id": "GO:0005334",
  "gene_name": "Sodium-dependent noradrenaline transporter",
  "gene_symbol": "SLC6A2"
}